{
  "gene": "UniProtKB:E2RYF7",
  "term_id": "UNKNOWN:0001",
  "term_label": "Unknown molecular function",
  "gene_symbol": "HCG22",
  "gene_name": "Protein PBMUCL2"
}